{
  "gene_symbol": "LMBR1L",
  "term_id": "GO:0007165",
  "gene_name": "Protein LMBR1L",
  "term_label": "signal transduction",
  "gene": "UniProtKB:Q6UX01"
}